{
  "gene_name": "SLIT and NTRK-like protein 5",
  "term_label": "axonogenesis",
  "gene_symbol": "SLITRK5",
  "gene": "UniProtKB:O94991",
  "term_id": "GO:0007409"
}